arachidonate 8(R)-lipoxygenase activity [GO:0047677] (molecular function) Note: This activity produces the R-enantiomer of HPETE, 8(R)-HPETE. For the reaction producing the S-enantiomer, see GO:0036403. Definition: Catalysis of the reaction: arachidonate + O2 = (5Z,8R,9E,11Z,14Z)-8-hydroperoxyicosa-5,9,11,14-tetraenoate. Also known as: arachidonate 8-lipoxygenase activity, 8-lipoxygenase activity, 8(R)-lipoxygenase activity, arachidonate:oxygen 8-oxidoreductase activity Sources: EC:1.13.11.40, RHEA:14985 Relationships: is a type of oxidoreductase activity, acting on single donors with incorporation of molecular oxygen, incorporation of two atoms of oxygen [GO:0016702]